{
  "gene": "UniProtKB:Q6DRA6",
  "term_id": "GO:0005634",
  "term_label": "nucleus",
  "gene_name": "Putative histone H2B type 2-D",
  "gene_symbol": "H2BC19P"
}